{
  "term_id": "GO:0005886",
  "term_label": "plasma membrane",
  "gene": "UniProtKB:O60637",
  "gene_symbol": "TSPAN3",
  "gene_name": "Tetraspanin-3"
}